{
  "gene_name": "Lipoprotein lipase",
  "gene": "UniProtKB:P06858",
  "term_id": "GO:0006633",
  "gene_symbol": "LPL",
  "term_label": "fatty acid biosynthetic process"
}